{
  "term_label": "extracellular matrix",
  "gene_name": "Collagen alpha-1(XI) chain",
  "term_id": "GO:0031012",
  "gene_symbol": "COL11A1",
  "gene": "UniProtKB:P12107"
}